{
  "gene_name": "Neuromedin-K receptor",
  "term_label": "tachykinin receptor activity",
  "gene_symbol": "TACR3",
  "gene": "UniProtKB:P29371",
  "term_id": "GO:0004995"
}